canonical inflammasome complex assembly [GO:0140632] (BP) Subtypes: NLRP3 inflammasome complex assembly [GO:0044546], CARD8 inflammasome complex assembly [GO:0140633], NLRP6 inflammasome complex assembly [GO:0140739], NLRP1 inflammasome complex assembly [GO:1904784] References: PMID:33420028, PMID:33420033, PMID:33542150 Relationships: is a type of protein-containing complex assembly [GO:0065003]; is part of inflammasome-mediated signaling pathway [GO:0141084] Definition: The aggregation, arrangement and bonding together of a set of components to form an inflammasome complex.